cellular response to sulfur dioxide [GO:0071252] (biological process) Sources: GOC:mah Definition: Any process that results in a change in state or activity of a cell (in terms of movement, secretion, enzyme production, gene expression, etc.) as a result of a sulfur dioxide (SO2) stimulus. Relationships: is a type of response to sulfur dioxide [GO:0010477]; is a type of GO:1901701